regulation of peroxisome organization [GO:1900063] (biological process) Relationships: is a type of regulation of organelle organization [GO:0033043]; regulates GO:0007031 Definition: Any process that modulates the frequency, rate or extent of peroxisome organization. Subtypes: positive regulation of peroxisome organization [GO:1900064] References: PMID:7500953 Sources: GOC:TermGenie Also known as: regulation of peroxisome organisation, regulation of peroxisome organization and biogenesis, regulation of peroxisome-assembly ATPase activity